cerebellar Purkinje cell-granule cell precursor cell signaling [GO:0021937] (BP) Relationships: is a type of cell-cell signaling [GO:0007267] References: PMID:15157725, PMID:32554107 Sources: GOC:cls, GOC:dgh, GOC:dph, GOC:jid, GO_REF:0000021 Definition: Any process that mediates the transfer of information from Purkinje cells to granule cell precursors.